{
  "term_id": "GO:0003723",
  "gene_symbol": "RPL6",
  "gene": "UniProtKB:Q02878",
  "term_label": "RNA binding",
  "gene_name": "Large ribosomal subunit protein eL6"
}